{
  "term_label": "B cell receptor signaling pathway",
  "gene_symbol": "CTLA4",
  "gene_name": "Cytotoxic T-lymphocyte protein 4",
  "term_id": "GO:0050853",
  "gene": "UniProtKB:P16410"
}